{
  "term_label": "amyloid-beta formation",
  "term_id": "GO:0034205",
  "gene_symbol": "PSEN2",
  "gene_name": "Presenilin-2",
  "gene": "UniProtKB:P49810"
}